{
  "gene_name": "Low-density lipoprotein receptor",
  "gene_symbol": "LDLR",
  "term_id": "GO:0042632",
  "term_label": "cholesterol homeostasis",
  "gene": "UniProtKB:P01130"
}